{
  "term_id": "GO:0000381",
  "term_label": "regulation of alternative mRNA splicing, via spliceosome",
  "gene_symbol": "RBM11",
  "gene_name": "Splicing regulator RBM11",
  "gene": "UniProtKB:P57052"
}